{
  "term_id": "GO:0005737",
  "gene_name": "Caveolae-associated protein 4",
  "term_label": "cytoplasm",
  "gene_symbol": "CAVIN4",
  "gene": "UniProtKB:Q5BKX8"
}